{
  "gene_name": "Zinc finger protein 461",
  "gene": "UniProtKB:Q8TAF7",
  "term_id": "GO:0005634",
  "term_label": "nucleus",
  "gene_symbol": "ZNF461"
}